{
  "term_id": "UNKNOWN:0001",
  "gene_name": "Prokineticin-2",
  "term_label": "Unknown molecular function",
  "gene": "UniProtKB:Q9HC23",
  "gene_symbol": "PROK2"
}